interleukin-7 binding [GO:0019982] (molecular function) Sources: GOC:jl Relationships: is a type of growth factor binding [GO:0019838]; is a type of GO:0019955 Also known as: IL-7 binding Definition: Binding to interleukin-7.